{
  "term_id": "GO:0035613",
  "gene_name": "Endogenous retrovirus group K member 10 Pol protein",
  "gene_symbol": "ERVK-10",
  "gene": "UniProtKB:P10266",
  "term_label": "RNA stem-loop binding"
}